{
  "gene_symbol": "ENTHD1",
  "term_label": "endosome",
  "gene": "UniProtKB:Q8IYW4",
  "term_id": "GO:0005768",
  "gene_name": "ENTH domain-containing protein 1"
}